{
  "gene_name": "Polypeptide N-acetylgalactosaminyltransferase-like 6",
  "term_label": "polypeptide N-acetylgalactosaminyltransferase activity",
  "term_id": "GO:0004653",
  "gene": "UniProtKB:Q49A17",
  "gene_symbol": "GALNTL6"
}